{
  "gene": "UniProtKB:Q99500",
  "gene_symbol": "S1PR3",
  "term_label": "G protein-coupled receptor activity",
  "gene_name": "Sphingosine 1-phosphate receptor 3",
  "term_id": "GO:0004930"
}